{
  "gene_name": "Calcium permeable stress-gated cation channel 1",
  "gene": "UniProtKB:Q9P1W3",
  "gene_symbol": "TMEM63C",
  "term_label": "Unknown biological process",
  "term_id": "UNKNOWN:0002"
}